{
  "gene_symbol": "SPG7",
  "term_id": "GO:0005745",
  "gene": "UniProtKB:Q9UQ90",
  "gene_name": "Paraplegin",
  "term_label": "m-AAA complex"
}